{
  "gene_symbol": "NUP214",
  "term_id": "GO:0017056",
  "gene_name": "Nuclear pore complex protein Nup214",
  "gene": "UniProtKB:P35658",
  "term_label": "structural constituent of nuclear pore"
}